positive regulation of mitotic sister chromatid separation [GO:1901970] (biological process) Definition: Any process that activates or increases the frequency, rate or extent of mitotic sister chromatid separation. Subtypes: GO:0045842, positive regulation of mitotic sister chromatid arm separation [GO:1905824] Also known as: activation of mitotic sister chromatid resolution, activation of sister chromatid separation during mitosis, positive regulation of mitotic sister chromatid resolution, positive regulation of sister chromatid separation during mitosis, up regulation of mitotic sister chromatid resolution, up regulation of mitotic sister chromatid separation, up regulation of sister chromatid separation during mitosis, up-regulation of mitotic sister chromatid resolution, up-regulation of mitotic sister chromatid separation, up-regulation of sister chromatid separation during mitosis, upregulation of mitotic sister chromatid resolution, upregulation of mitotic sister chromatid separation, upregulation of sister chromatid separation during mitosis, activation of mitotic sister chromatid separation, activation of chromosome separation during mitosis, activation of mitotic chromosome separation, positive regulation of chromosome separation during mitosis, positive regulation of mitotic chromosome separation, up regulation of chromosome separation during mitosis, up regulation of mitotic chromosome separation, up-regulation of chromosome separation during mitosis, up-regulation of mitotic chromosome separation, upregulation of chromosome separation during mitosis, upregulation of mitotic chromosome separation Relationships: is a type of GO:0010965; is a type of positive regulation of chromosome separation [GO:1905820]; RO_0002213 mitotic sister chromatid separation [GO:0051306] References: PMID:1846086 Sources: GOC:TermGenie